cardiac skeleton development [GO:0003204] (biological process) Relationships: is a type of connective tissue development [GO:0061448]; is part of heart development [GO:0007507] Definition: The progression of the cardiac skeleton over time, from its formation to the mature structure. The cardiac skeleton is a specialized extracellular matrix that separates the atria from the ventricles and provides physical support for the heart. Sources: GOC:mtg_heart Also known as: heart fibrous skeleton development